{
  "gene_symbol": "RPS23",
  "gene": "UniProtKB:P62266",
  "gene_name": "Small ribosomal subunit protein uS12",
  "term_id": "GO:0006412",
  "term_label": "translation"
}